{
  "gene_name": "GPI ethanolamine phosphate transferase 2",
  "gene_symbol": "PIGG",
  "term_label": "CP2 mannose-ethanolamine phosphotransferase activity",
  "gene": "UniProtKB:Q5H8A4",
  "term_id": "GO:0051267"
}